{
  "term_label": "olfactory receptor activity",
  "gene": "UniProtKB:O95221",
  "gene_name": "Olfactory receptor 5F1",
  "term_id": "GO:0004984",
  "gene_symbol": "OR5F1"
}